{
  "gene": "UniProtKB:Q14576",
  "gene_name": "ELAV-like protein 3",
  "term_label": "Unknown biological process",
  "term_id": "UNKNOWN:0002",
  "gene_symbol": "ELAVL3"
}